ripoptosome assembly involved in extrinsic apoptotic signaling pathway [GO:1901025] (biological process) References: PMID:22274400 Sources: GOC:TermGenie, GOC:mtg_apoptosis Relationships: is a type of ripoptosome assembly [GO:0097343]; is part of extrinsic apoptotic signaling pathway [GO:0097191] Definition: The aggregation, arrangement and bonding together of ripoptosome components leading to apoptosis via the extrinsic apoptotic signaling pathway.